{
  "term_id": "GO:0009313",
  "term_label": "oligosaccharide catabolic process",
  "gene_symbol": "NEU1",
  "gene": "UniProtKB:Q99519",
  "gene_name": "Sialidase-1"
}